molecular function inhibitor activity [GO:0140678] (molecular function) Relationships: is a type of molecular function regulator activity [GO:0098772] Sources: GOC:curators Definition: A molecular function regulator that inhibits or decreases the activity of its target via non-covalent binding that does not result in covalent modification to the target. Note: This term should only be used in cases when the regulator directly interacts with the enzyme, but does not result in a covalent modification. Subtypes: enzyme inhibitor activity [GO:0004857], signaling receptor inhibitor activity [GO:0030547], GO:0042030, transcription regulator inhibitor activity [GO:0140416], cytoskeletal motor inhibitor activity [GO:0140661], miRNA inhibitor activity via base-pairing [GO:0140869], GO:0140871, receptor ligand inhibitor activity [GO:0141069], transporter inhibitor activity [GO:0141110]